{
  "gene": "UniProtKB:P68366",
  "term_label": "microtubule cytoskeleton organization",
  "term_id": "GO:0000226",
  "gene_name": "Tubulin alpha-4A chain",
  "gene_symbol": "TUBA4A"
}